{
  "term_label": "sensory perception of sound",
  "gene": "UniProtKB:Q8WXG9",
  "term_id": "GO:0007605",
  "gene_symbol": "ADGRV1",
  "gene_name": "Adhesion G-protein coupled receptor V1"
}